5-carbamoylmethyl uridine residue modification [GO:0080178] (biological process) Relationships: is a type of tRNA methylation [GO:0030488] Sources: GOC:dph, GOC:tb Definition: The chemical reactions and pathways involving the addition of a 5-carbamoylmethyl group to a uridine residue in RNA. Also known as: 5-carbamoylmethyluridine metabolic process